chromosomal 5-methylcytosine DNA demethylation, oxidation pathway [GO:0141167] (biological process) Also known as: epigenetic 5-methylcytosine DNA demethylation, oxidation pathway, epigenetic DNA demethylation, oxidation pathway Note: Note that this term describes one of the biochemical pathways of chromosomal cytosine demethylation but is agnostic to the effect on gene expression. If the data supports it, consider co-annotating to 'positive regulation of gene expression, epigenetic ; GO:0044029' or a child. A similar pathway may also convert chromosomal DNA N6-methyladenosine to adenosine but little evidence exists for this pathway. References: PMID:21862972, PMID:29875631, PMID:36478523 Relationships: is a type of GO:0141137; is a type of chromosomal 5-methylcytosine DNA demethylation pathway [GO:0141166] Definition: An epigenetic cytosine DNA demethylation pathway that starts with the enzymatic oxidation of the 5-methylcytosine (5meC) to generate 5-hydroxymethylcytosine (5hmC), which successively converted to 5-formylcytosine (5fC) and 5-carboxylcytosine (5caC).  A DNA glycosylase (e. g. TDG) recognizes the  intermediate bases 5fC and 5caC and excises the modified base to initiate its replacement with unmethylated cytosine through base excision repair.